{
  "term_label": "nervous system development",
  "gene_symbol": "NRXN3",
  "gene_name": "Neurexin-3",
  "term_id": "GO:0007399",
  "gene": "UniProtKB:Q9Y4C0"
}